dinoflagellate apex [GO:0097683] (cellular component) References: PMID:7002229 Sources: GOC:at, Wikipedia:Dinoflagellate#Morphology, http://tolweb.org/Dinoflagellates/2445 Relationships: is a type of cellular anatomical structure [GO:0110165]; is part of GO:0097613 Subtypes: dinoflagellate apical horn [GO:0097686] Also known as: apex Note: The term name refers to a taxonomic group to make the label unique with respect to similarly-named anatomical structures. Definition: The anterior most point of a dinoflagellate epicone.